cytoplasmic side of trans-Golgi cisterna membrane [GO:0160288] (cellular component) Relationships: is a type of cytoplasmic side of membrane [GO:0098562]; is part of GO:1990676 References: PMID:23913272, PMID:34597626, PMID:37566051 Definition: The membrane leaflet of the trans-Golgi cisternae that faces the cytoplasm. It is the site of protein and lipid interaction, vesicle formation, and cargo sorting towards post-Golgi destinations such as endosomes, lysosomes, and the plasma membrane. Also known as: cytoplasmic face of Golgi trans cisterna membrane, cytoplasmic leaflet of Golgi trans cisterna membrane, cytoplasmic side of Golgi trans cisternae membrane